{
  "term_id": "UNKNOWN:0003",
  "gene_name": "Ral GTPase-activating protein subunit beta",
  "gene_symbol": "RALGAPB",
  "gene": "UniProtKB:Q86X10",
  "term_label": "Unknown cellular component"
}